{
  "gene_symbol": "SLC22A5",
  "term_label": "quaternary ammonium group transport",
  "term_id": "GO:0015697",
  "gene": "UniProtKB:O76082",
  "gene_name": "Organic cation_carnitine transporter 2"
}